{
  "gene": "UniProtKB:Q96T58",
  "gene_symbol": "SPEN",
  "term_id": "GO:0003729",
  "gene_name": "Msx2-interacting protein",
  "term_label": "mRNA binding"
}